head kidney structural organization [GO:0072119] (biological process) Relationships: is a type of pronephros structural organization [GO:0072118]; is part of head kidney morphogenesis [GO:0072115] Sources: GOC:mtg_kidney_jan10, ZFA:0000669 Also known as: head kidney structural organisation Definition: The process that contributes to the act of creating the structural organization of the head kidney. This process pertains to the physical shaping of a rudimentary structure. The head kidney is a pronephros that consists of fused bilateral lobes located in the anterior part of the kidney.